{
  "term_id": "UNKNOWN:0003",
  "gene_symbol": "PYCR3",
  "term_label": "Unknown cellular component",
  "gene": "UniProtKB:Q53H96",
  "gene_name": "Pyrroline-5-carboxylate reductase 3"
}